{
  "gene": "UniProtKB:Q8IXV7",
  "gene_name": "Kelch domain-containing protein 8B",
  "gene_symbol": "KLHDC8B",
  "term_label": "nuclear chromosome segregation",
  "term_id": "GO:0098813"
}